{
  "term_label": "Unknown biological process",
  "term_id": "UNKNOWN:0002",
  "gene_name": "Uncharacterized protein",
  "gene_symbol": "A0A8I5KPI3",
  "gene": "UniProtKB:A0A8I5KPI3"
}